{
  "gene": "UniProtKB:P50607",
  "gene_name": "Tubby protein homolog",
  "gene_symbol": "TUB",
  "term_label": "protein localization to cilium",
  "term_id": "GO:0061512"
}